ADP:phosphate antiporter activity [GO:0140988] (molecular function) Relationships: is a type of GO:0015217; is a type of organophosphate:phosphate antiporter activity [GO:0015315] Also known as: ADP:inorganic phosphate antiporter activity, inorganic phosphate:ADP antiporter activity Definition: Enables the transfer of ADP from one side of a membrane to the other according to the reaction: ADP(out) + phosphate(in) = ADP(in) + phosphate(out). References: PMID:15123600